adrenal cortex development [GO:0035801] (biological process) Relationships: is a type of anatomical structure development [GO:0048856]; is part of adrenal gland development [GO:0030325] Definition: The process whose specific outcome is the progression of the adrenal cortex over time, from its formation to the mature structure. The adrenal cortex is located at the periphery of the adrenal gland and controls glucose and electrolyte metabolism, response to stress and sexual development through the production of different classes of steroid hormones (glucocorticoids, mineralocorticoids and androgens). Also known as: adrenal gland cortex development References: PMID:12185666, PMID:21115154 Sources: Wikipedia:Adrenal_cortex